5S rRNA binding [GO:0008097] (molecular function) Definition: Binding to a 5S ribosomal RNA, the smallest RNA constituent of a ribosome. Relationships: is a type of rRNA binding [GO:0019843] Sources: GOC:jl, ISBN:0321000382 Subtypes: 5S rRNA primary transcript binding [GO:0008098]